cordyol C biosynthetic process [GO:1900799] (biological process) Also known as: cordyol C anabolism, cordyol C biosynthesis, cordyol C formation, cordyol C synthesis Relationships: is_a catechol-containing compound biosynthetic process [GO:0009713]; is a type of secondary metabolite biosynthetic process [GO:0044550]; is a type of cordyol C metabolic process [GO:1900797]; is a type of ether biosynthetic process [GO:1901503] Definition: The chemical reactions and pathways resulting in the formation of cordyol C. Sources: GOC:TermGenie, GOC:di Regulation: regulated by regulation of cordyol C biosynthetic process [GO:1900861]; negatively regulated by negative regulation of cordyol C biosynthetic process [GO:1900862]; positively regulated by positive regulation of cordyol C biosynthetic process [GO:1900863]